{
  "term_id": "GO:0003689",
  "gene_symbol": "RFC5",
  "gene": "UniProtKB:P40937",
  "term_label": "DNA clamp loader activity",
  "gene_name": "Replication factor C subunit 5"
}